{
  "term_label": "skeletal system morphogenesis",
  "gene_name": "Collagen alpha-3(V) chain",
  "term_id": "GO:0048705",
  "gene": "UniProtKB:P25940",
  "gene_symbol": "COL5A3"
}